{
  "term_id": "UNKNOWN:0001",
  "term_label": "Unknown molecular function",
  "gene_name": "COP9 signalosome complex subunit 9",
  "gene": "UniProtKB:Q8WXC6",
  "gene_symbol": "COPS9"
}